nucleolar chromatin [GO:0030874] (cellular component) Subtypes: GO:0005731, nucleolus-associated heterochromatin [GO:0097424] Relationships: is a type of chromatin [GO:0000785]; is part of nuclear chromosome [GO:0000228]; is part of nucleolus [GO:0005730] Definition: The portion of nuclear chromatin associated with the nucleolus; includes the DNA encoding the ribosomal RNA. Sources: GOC:mah